{
  "gene_symbol": "SRC",
  "gene": "UniProtKB:P12931",
  "term_id": "GO:0005102",
  "term_label": "signaling receptor binding",
  "gene_name": "Proto-oncogene tyrosine-protein kinase Src"
}